low-density lipoprotein particle receptor catabolic process [GO:0032802] (biological process) Sources: GOC:mah Definition: The chemical reactions and pathways resulting in the breakdown of a low-density lipoprotein particle receptor molecule, a macromolecule that undergoes combination with a hormone, neurotransmitter, drug or intracellular messenger to initiate a change in cell function. Relationships: is a type of protein catabolic process [GO:0030163]; is a type of GO:0032799; is a type of receptor catabolic process [GO:0032801] Regulation: regulated by regulation of low-density lipoprotein particle receptor catabolic process [GO:0032803]; negatively regulated by negative regulation of low-density lipoprotein particle receptor catabolic process [GO:0032804]; positively regulated by positive regulation of low-density lipoprotein particle receptor catabolic process [GO:0032805] Also known as: LDL receptor breakdown, LDL receptor catabolic process, LDL receptor degradation, low-density lipoprotein receptor breakdown, low-density lipoprotein receptor catabolic process, low-density lipoprotein receptor catabolism, low-density lipoprotein receptor degradation, LDL receptor catabolism